chromatin [GO:0000785] (cellular component) Note: Chromosomes include parts that are not part of the chromatin. Examples include the kinetochore. References: PMID:20404130 Sources: GOC:elh Subtypes: GO:0000791, GO:0000792, GO:0030874, CENP-A containing chromatin [GO:0061638] Relationships: is a type of cellular anatomical structure [GO:0110165]; is part of chromosome [GO:0005694] Also known as: cytoplasmic chromatin, nuclear chromatin, chromosome scaffold Definition: The ordered and organized complex of DNA, protein, and sometimes RNA, that forms the chromosome.